CD4-positive, alpha-beta T cell activation [GO:0035710] (biological process) Sources: CL:0000624, GOC:BHF Relationships: is_a GO:0046631 Definition: The change in morphology and behavior of a CD4-positive, alpha-beta T cell resulting from exposure to a mitogen, cytokine, chemokine, cellular ligand, or an antigen for which it is specific. Regulation: regulated by GO:2000514; negatively regulated by negative regulation of CD4-positive, alpha-beta T cell activation [GO:2000515]; positively regulated by GO:2000516 Subtypes: GO:0035711, T-helper 2 cell activation [GO:0035712], CD4-positive, alpha-beta T cell proliferation [GO:0035739], CD4-positive, alpha-beta T cell differentiation [GO:0043367]